cytidine to uridine editing [GO:0016554] (biological process) Definition: The conversion of a cytosine residue to uridine in an RNA molecule by deamination. References: PMID:11092837 Relationships: is a type of base conversion or substitution editing [GO:0016553]